renal system process involved in regulation of blood volume [GO:0001977] (biological process) Definition: A slow mechanism of blood pressure regulation that responds to changes in pressure resulting from fluid and salt intake by modulating the quantity of blood in the circulatory system. Sources: GOC:dph, GOC:tb, ISBN:0721643949 Also known as: renal blood volume control of blood pressure, renal regulation of blood volume Relationships: is a type of renal system process involved in regulation of systemic arterial blood pressure [GO:0003071]; is part of regulation of body fluid levels [GO:0050878] Subtypes: GO:0002017, regulation of glomerular filtration [GO:0003093], pressure natriuresis [GO:0003095], tubuloglomerular feedback [GO:0003098]